protein-N(PI)-phosphohistidine-D-glucosamine phosphotransferase system transporter activity [GO:0090590] (molecular function) Definition: Catalysis of the PEP-dependent, phosphoryl transfer-driven transport of substances across a membrane. The transport happens by catalysis of the reaction: protein N-phosphohistidine + D-glucosamine(out) = protein histidine + glucosamine-6-phosphate(in). References: PMID:8246840 Relationships: is_a protein-N(PI)-phosphohistidine-sugar phosphotransferase activity [GO:0008982]